host cell nuclear inner membrane [GO:0044201] (cellular component) Relationships: is a type of host cell nuclear membrane [GO:0044200] Definition: The inner, i.e. lumen-facing, lipid bilayer of the host nuclear envelope. Sources: GOC:jl